{
  "gene": "UniProtKB:Q6ZWC4",
  "gene_name": "Putative uncharacterized protein LOC100128429",
  "term_id": "UNKNOWN:0002",
  "term_label": "Unknown biological process",
  "gene_symbol": "Q6ZWC4"
}